{
  "gene_symbol": "ULK3",
  "gene_name": "Serine_threonine-protein kinase ULK3",
  "term_label": "autophagosome",
  "gene": "UniProtKB:Q6PHR2",
  "term_id": "GO:0005776"
}